{
  "term_id": "UNKNOWN:0003",
  "term_label": "Unknown cellular component",
  "gene_symbol": "ZNF502",
  "gene_name": "Zinc finger protein 502",
  "gene": "UniProtKB:Q8TBZ5"
}